interleukin-28A production [GO:0072627] (biological process) Relationships: is a type of type III interferon production [GO:0034343] Also known as: IL-28A production, IL28A production, interferon lambda 2 production, interleukin-28A secretion Note: Note that this term is in the subset of terms that should not be used for direct gene product annotation. Instead, select one of the 'regulation' children terms. Definition: The appearance of interleukin-28A due to biosynthesis or secretion following a cellular stimulus, resulting in an increase in its intracellular or extracellular levels. References: PMID:15546383 Sources: GOC:BHF, GOC:mah